Notch receptor processing, ligand-independent [GO:0035334] (biological process) Also known as: Notch S1 cleavage Definition: The proteolytic cleavages to the Notch protein that occur prior to ligand binding. A primary cleavage event within the extracellular domain whilst the Notch protein in still in the secretory pathway, leads to the transportation of a processed heterodimer to the cell surface. Relationships: is_a protein processing [GO:0016485]; BFO_0000050 Notch receptor processing [GO:0007220] References: PMID:12651094 Sources: GOC:bf